{
  "gene_symbol": "GDF15",
  "gene": "UniProtKB:Q99988",
  "term_label": "cell surface receptor protein serine/threonine kinase signaling pathway",
  "term_id": "GO:0007178",
  "gene_name": "Growth_differentiation factor 15"
}